protein N-acetylglucosaminyltransferase complex [GO:0017122] (cellular component) Relationships: is a type of intracellular protein-containing complex [GO:0140535]; is a type of transferase complex [GO:1990234] Definition: A protein complex capable of protein N-acetylglucosaminyltransferase activity, the addition of nucleotide-activated sugars onto the polypeptide according to reaction: UDP-N-acetyl-D-glucosamine + protein = UDP + 4-N-(N-acetyl-D-glucosaminyl)-protein. The complex has different compositions in different species: In mammals it is often a homotrimer, in bacteria a heterotetramer of 2 different subunits. Also known as: O-GlcNAc transferase complex, UDP-N-acetylglucosamine-peptide N-acetylglucosaminyltransferase References: PMID:15247246